{
  "gene_symbol": "OR1P1",
  "term_id": "GO:0005886",
  "term_label": "plasma membrane",
  "gene_name": "Olfactory receptor 1P1",
  "gene": "UniProtKB:Q8NH06"
}